glycoprotein 2-beta-D-xylosyltransferase activity [GO:0050513] (molecular function) Also known as: glycoprotein 2-b-D-xylosyltransferase activity, 1,2-beta-xylosyltransferase activity, beta-1,2-xylosyltransferase activity Definition: Catalysis of the reaction: N(4)-{N-acetyl-beta-D-glucosaminyl-(1->2)-alpha-D-mannosyl-(1->3)-[N-acetyl-beta-D-glucosaminyl-(1->2)-alpha-D-mannosyl-(1->6)]-beta-D-mannosyl-(1->4)-N-acetyl-beta-D-glucosaminyl-(1->4)-N-acetyl-beta-D-glucosaminyl}-L-asparagine + UDP-alpha-D-xylose = N(4)-{N-acetyl-beta-D-glucosaminyl-(1->2)-alpha-D-mannosyl-(1->3)-[N-acetyl-beta-D-glucosaminyl-(1->2)-alpha-D-mannosyl-(1->6)]-[beta-D-xylosyl-(1->2)]-beta-D-mannosyl-(1->4)-N-acetyl-beta-D-glucosaminyl-(1->4)-N-acetyl-beta-D-glucosaminyl}-L-asparagine + H+ + UDP. Relationships: is a type of GO:0035252 Sources: EC:2.4.2.38, RHEA:10612